regulation of translational initiation [GO:0006446] (biological process) Subtypes: GO:0006447, regulation of eIF2 alpha phosphorylation by heme [GO:0010999], GO:0043558, negative regulation of translational initiation [GO:0045947], positive regulation of translational initiation [GO:0045948], regulation of endoplasmic reticulum stress-induced eIF2 alpha phosphorylation [GO:0060734], GO:0060735, GO:0070132, negative regulation of endoplasmic reticulum stress-induced eIF2 alpha phosphorylation [GO:1903912], GO:1904688, regulation of translational initiation by tRNA modification [GO:1990983] Sources: GOC:go_curators Definition: Any process that modulates the frequency, rate or extent of translational initiation. Relationships: is a type of GO:0006417; regulates GO:0006413